{
  "term_label": "positive regulation of transcription by RNA polymerase II",
  "term_id": "GO:0045944",
  "gene": "UniProtKB:P41225",
  "gene_symbol": "SOX3",
  "gene_name": "Transcription factor SOX-3"
}